2-hydroxy-3-oxopropionate reductase activity [GO:0008679] (molecular function) Definition: Catalysis of the reaction: (R)-glycerate + NADP+ = 2-hydroxy-3-oxopropanoate + NADPH + H+. Sources: EC:1.1.1.60 Also known as: (R)-glycerate:NAD(P)+ oxidoreductase activity, tartronate semialdehyde reductase (NADPH) activity Relationships: is a type of GO:0016616